{
  "term_label": "receptor tyrosine kinase binding",
  "gene": "UniProtKB:O15123",
  "gene_name": "Angiopoietin-2",
  "gene_symbol": "ANGPT2",
  "term_id": "GO:0030971"
}